{
  "term_label": "DNA binding",
  "gene": "UniProtKB:Q63HK5",
  "term_id": "GO:0003677",
  "gene_symbol": "TSHZ3",
  "gene_name": "Teashirt homolog 3"
}